regulation of myotube cell migration [GO:0110123] (biological process) Definition: Any process that modulates the frequency, rate or extent of myotube cell migration. Relationships: is a type of regulation of cell migration [GO:0030334]; RO_0002211 myotube cell migration [GO:0110122] References: PMID:29122742 Sources: GOC:ha Subtypes: positive regulation of myotube cell migration [GO:0110124], negative regulation of myotube cell migration [GO:0110125]